{
  "gene_symbol": "SLC4A9",
  "term_id": "GO:0008510",
  "gene": "UniProtKB:Q96Q91",
  "term_label": "sodium:bicarbonate symporter activity",
  "gene_name": "Anion exchange protein 4"
}